{
  "gene_name": "Protein fem-1 homolog C",
  "term_label": "proteasome-mediated ubiquitin-dependent protein catabolic process",
  "gene_symbol": "FEM1C",
  "term_id": "GO:0043161",
  "gene": "UniProtKB:Q96JP0"
}